{
  "term_label": "oxidoreductase activity",
  "term_id": "GO:0016491",
  "gene": "UniProtKB:Q7Z5J1",
  "gene_symbol": "HSD11B1L",
  "gene_name": "Hydroxysteroid 11-beta-dehydrogenase 1-like protein"
}